{
  "term_id": "GO:0006537",
  "gene_symbol": "GLS2",
  "term_label": "glutamate biosynthetic process",
  "gene": "UniProtKB:Q9UI32",
  "gene_name": "Glutaminase liver isoform, mitochondrial"
}